transforming growth factor beta1 production [GO:0032905] (biological process) Also known as: TGF-B1 production, TGFB1 production, transforming growth factor-beta1 production Definition: The appearance of transforming growth factor-beta1 due to biosynthesis or secretion following a cellular stimulus, resulting in an increase in its intracellular or extracellular levels. Relationships: is a type of transforming growth factor beta production [GO:0071604] Sources: GOC:mah Regulation: regulated by regulation of transforming growth factor beta1 production [GO:0032908]; negatively regulated by GO:0032911; positively regulated by GO:0032914